{
  "term_label": "nucleus",
  "gene_name": "DNA-(apurinic or apyrimidinic site) endonuclease 2",
  "gene": "UniProtKB:Q9UBZ4",
  "gene_symbol": "APEX2",
  "term_id": "GO:0005634"
}